{
  "term_label": "Unknown molecular function",
  "gene_symbol": "HAPLN2",
  "gene": "UniProtKB:Q9GZV7",
  "gene_name": "Hyaluronan and proteoglycan link protein 2",
  "term_id": "UNKNOWN:0001"
}